{
  "gene_symbol": "OCEL1",
  "term_id": "GO:0005923",
  "gene_name": "Occludin_ELL domain-containing protein 1",
  "term_label": "bicellular tight junction",
  "gene": "UniProtKB:Q9H607"
}